regulation of adaptive immune response [GO:0002819] (biological process) Relationships: is a type of regulation of immune response [GO:0050776]; RO_0002211 adaptive immune response [GO:0002250] Definition: Any process that modulates the frequency, rate, or extent of an adaptive immune response. Subtypes: negative regulation of adaptive immune response [GO:0002820], positive regulation of adaptive immune response [GO:0002821], regulation of adaptive immune response based on somatic recombination of immune receptors built from immunoglobulin superfamily domains [GO:0002822], regulation of adaptive immune memory response [GO:1905674], regulation of adaptive immune effector response [GO:1905677] Sources: GOC:add